{
  "term_id": "GO:0000045",
  "gene_name": "Syntaxin-12",
  "gene": "UniProtKB:Q86Y82",
  "gene_symbol": "STX12",
  "term_label": "autophagosome assembly"
}